pyrimidine deoxyribonucleotide biosynthetic process [GO:0009221] (biological process) Definition: The chemical reactions and pathways resulting in the formation of a pyrimidine deoxyribonucleotide, a compound consisting of nucleoside (a pyrimidine base linked to a deoxyribose sugar) esterified with a phosphate group at either the 3' or 5'-hydroxyl group of the sugar. Sources: GOC:go_curators, ISBN:0198506732 Relationships: is a type of pyrimidine nucleotide biosynthetic process [GO:0006221]; is_a pyrimidine deoxyribonucleotide metabolic process [GO:0009219]; is a type of 2'-deoxyribonucleotide biosynthetic process [GO:0009265] Subtypes: GO:0006226, dUDP biosynthetic process [GO:0006227], dUTP biosynthetic process [GO:0006229], GO:0006231, dTDP biosynthetic process [GO:0006233], dTTP biosynthetic process [GO:0006235], dCDP biosynthetic process [GO:0006240], dCTP biosynthetic process [GO:0006242], pyrimidine deoxyribonucleotide salvage [GO:0010139], dCMP biosynthetic process [GO:0046064] Also known as: pyrimidine deoxyribonucleotide anabolism, pyrimidine deoxyribonucleotide biosynthesis, pyrimidine deoxyribonucleotide formation, pyrimidine deoxyribonucleotide synthesis